{
  "term_label": "protein exit from endoplasmic reticulum",
  "gene_name": "Protein SEC13 homolog",
  "gene_symbol": "SEC13",
  "term_id": "GO:0032527",
  "gene": "UniProtKB:P55735"
}